bacterial-type DNA replication termination [GO:1902329] (biological process) Definition: Any DNA replication termination that is involved in bacterial-type DNA replication. Sources: GOC:TermGenie, GOC:mtg_cell_cycle Also known as: DNA replication termination involved in bacterial-type DNA replication Relationships: is a type of cell cycle DNA replication termination [GO:1902294]; is part of bacterial-type DNA replication [GO:0044787]